intercalary leaflet morphogenesis [GO:0060780] (biological process) Definition: The process in which the intercalary leaflet attains its shape. An intercalary leaflet is a leaflet that develops between primary leaflets. Relationships: is a type of GO:0060794 Sources: GOC:dph, GOC:sdb_2009, GOC:tb